{
  "term_label": "neuron development",
  "gene": "UniProtKB:P0C7M4",
  "gene_name": "Rhox homeobox family member 2B",
  "term_id": "GO:0048666",
  "gene_symbol": "RHOXF2B"
}